{
  "gene": "UniProtKB:Q08334",
  "gene_symbol": "IL10RB",
  "term_label": "interleukin-10 receptor activity",
  "gene_name": "Interleukin-10 receptor subunit beta",
  "term_id": "GO:0004920"
}